{
  "gene_name": "V-set and transmembrane domain-containing protein 2A",
  "gene_symbol": "VSTM2A",
  "term_label": "Unknown molecular function",
  "term_id": "UNKNOWN:0001",
  "gene": "UniProtKB:Q8TAG5"
}